{
  "gene": "UniProtKB:A6NMX2",
  "gene_symbol": "EIF4E1B",
  "term_id": "GO:0016281",
  "gene_name": "Eukaryotic translation initiation factor 4E type 1B",
  "term_label": "eukaryotic translation initiation factor 4F complex"
}